glutathione import across plasma membrane [GO:0098709] (biological process) Relationships: is a type of glutathione transmembrane transport [GO:0034775]; is a type of tripeptide import across plasma membrane [GO:0140207] Sources: GOC:dos Also known as: glutathione import into cell, glutathione uptake Definition: The directed movement of glutathione from outside of a cell, across the plasma membrane and into the cytosol.